{
  "term_label": "ciliary basal body",
  "gene_symbol": "CEP41",
  "gene_name": "Centrosomal protein of 41 kDa",
  "gene": "UniProtKB:Q9BYV8",
  "term_id": "GO:0036064"
}